{
  "gene": "UniProtKB:Q3KNV8",
  "gene_symbol": "PCGF3",
  "term_label": "PRC1 complex",
  "term_id": "GO:0035102",
  "gene_name": "Polycomb group RING finger protein 3"
}